{
  "gene": "UniProtKB:P02788",
  "term_label": "iron ion transport",
  "gene_symbol": "LTF",
  "gene_name": "Lactotransferrin",
  "term_id": "GO:0006826"
}